{
  "gene": "UniProtKB:P32248",
  "gene_symbol": "CCR7",
  "gene_name": "C-C chemokine receptor type 7",
  "term_id": "GO:0007204",
  "term_label": "positive regulation of cytosolic calcium ion concentration"
}